{
  "gene": "UniProtKB:P13378",
  "term_label": "nucleus",
  "term_id": "GO:0005634",
  "gene_name": "Homeobox protein Hox-D8",
  "gene_symbol": "HOXD8"
}